{
  "gene": "UniProtKB:P62330",
  "gene_name": "ADP-ribosylation factor 6",
  "gene_symbol": "ARF6",
  "term_label": "GTP binding",
  "term_id": "GO:0005525"
}